discadenine synthase activity [GO:0047870] (MF) Relationships: is a type of transferase activity, transferring alkyl or aryl (other than methyl) groups [GO:0016765] Sources: EC:2.5.1.24, RHEA:19581 Definition: Catalysis of the reaction: N(6)-dimethylallyladenine + S-adenosyl-L-methionine(1+) = S-methyl-5'-thioadenosine + discadenine + H+. Also known as: S-adenosyl-L-methionine:6-N-(Delta2-isopentenyl)-adenine 3-(3-amino-3-carboxypropyl)-transferase activity, S-adenosyl-L-methionine:N6-(Delta2-isopentenyl)-adenine 3-(3-amino-3-carboxypropyl)-transferas, discadenine synthetase activity